{
  "gene": "UniProtKB:P06748",
  "term_id": "GO:0005730",
  "gene_name": "Nucleophosmin",
  "gene_symbol": "NPM1",
  "term_label": "nucleolus"
}